F-actin capping protein complex [GO:0008290] (cellular component) Relationships: is a type of protein-containing complex [GO:0032991]; is part of actin cytoskeleton [GO:0015629] Sources: GOC:go_curators, ISBN:0198599560 Definition: A heterodimer consisting of alpha and beta subunits that binds to and caps the barbed ends of actin filaments, thereby regulating the polymerization of actin monomers but not severing actin filaments. Subtypes: actin capping protein of dynactin complex [GO:0005870]